{
  "gene_symbol": "VPS18",
  "term_id": "GO:0030674",
  "gene_name": "Vacuolar protein sorting-associated protein 18 homolog",
  "term_label": "protein-macromolecule adaptor activity",
  "gene": "UniProtKB:Q9P253"
}